{
  "term_label": "Unknown molecular function",
  "gene_symbol": "CEACAM18",
  "gene": "UniProtKB:A8MTB9",
  "gene_name": "Carcinoembryonic antigen-related cell adhesion molecule 18",
  "term_id": "UNKNOWN:0001"
}